cyclin K-CDK12 complex [GO:0002944] (cellular component) Also known as: CycK/Cdk12 complex References: PMID:22012619 Relationships: is a type of cyclin-dependent protein kinase holoenzyme complex [GO:0000307] Definition: A protein complex consisting of cyclin Kand cyclin-dependent kinase 12 (CDK12). Cyclins are characterized by periodicity in protein abundance throughout the cell cycle. Cyclin-dependent kinases represent a family of serine/threonine protein kinases that become active upon binding to a cyclin regulatory partner.